{
  "gene_symbol": "MPZL2",
  "term_label": "cell-cell adhesion",
  "gene": "UniProtKB:O60487",
  "term_id": "GO:0098609",
  "gene_name": "Myelin protein zero-like protein 2"
}